{
  "gene_name": "ADP_ATP translocase 3",
  "gene_symbol": "SLC25A6",
  "term_id": "GO:1990544",
  "term_label": "mitochondrial ATP transmembrane transport",
  "gene": "UniProtKB:P12236"
}